vesicle tethering [GO:0099022] (biological process) Subtypes: vesicle tethering involved in exocytosis [GO:0090522], vesicle tethering to Golgi [GO:0099041], GO:0099044 Relationships: is a type of cellular component organization [GO:0016043]; is part of vesicle targeting [GO:0006903] Definition: The initial, indirect interaction between a vesicle membrane and a membrane to which it is targeted for fusion. This interaction is mediated by tethering factors (or complexes), which interact with both membranes. Interaction can occur via direct binding to membrane phospholipids or membrane proteins, or via binding to vesicle coat proteins. This process is distinct from and prior to interaction between factors involved in fusion. References: PMID:27243008